UDP-D-xylose metabolic process [GO:0033319] (biological process) Also known as: UDP-D-xylose metabolism Definition: The chemical reactions and pathways involving UDP-D-xylose, uridinediphosphoxylose, a substance composed of xylose in glycosidic linkage with uridine diphosphate. Sources: GOC:mah Subtypes: GO:0033320 Relationships: is a type of nucleotide-sugar metabolic process [GO:0009225]